{
  "gene_symbol": "ERVK-21",
  "gene": "UniProtKB:P61565",
  "gene_name": "Endogenous retrovirus group K member 21 Env polyprotein",
  "term_label": "Unknown cellular component",
  "term_id": "UNKNOWN:0003"
}